{
  "term_label": "Unknown biological process",
  "gene": "UniProtKB:Q9UMZ2",
  "gene_name": "Synergin gamma",
  "gene_symbol": "SYNRG",
  "term_id": "UNKNOWN:0002"
}